{
  "gene_name": "Low affinity immunoglobulin gamma Fc region receptor III-A",
  "gene": "UniProtKB:P08637",
  "term_id": "GO:0001788",
  "term_label": "antibody-dependent cellular cytotoxicity",
  "gene_symbol": "FCGR3A"
}